{
  "gene_symbol": "SPECC1",
  "gene": "UniProtKB:Q5M775",
  "gene_name": "Cytospin-B",
  "term_label": "Unknown molecular function",
  "term_id": "UNKNOWN:0001"
}